{
  "term_label": "nucleate erythrocyte development",
  "gene_name": "Small integral membrane protein 1",
  "gene_symbol": "SMIM1",
  "gene": "UniProtKB:B2RUZ4",
  "term_id": "GO:0048823"
}